mammillothalamic axonal tract development [GO:0061374] (biological process) Definition: The progression of the mammillothalamic axonal tract, from its formation to the mature structure. The mammillothalamic tract is the collection of axons that connects the two major subdivisions of the diencephalon (hypothalamus and thalamus) and closes the diencephalic circuit. References: PMID:10662642 Sources: GOC:dph, GOC:yaf Relationships: is a type of anatomical structure development [GO:0048856]; BFO_0000050 mammillary axonal complex development [GO:0061373]